{
  "term_id": "GO:0070822",
  "gene_symbol": "SAP130",
  "gene_name": "Histone deacetylase complex subunit SAP130",
  "term_label": "Sin3-type complex",
  "gene": "UniProtKB:Q9H0E3"
}